{
  "term_id": "GO:0016791",
  "gene": "UniProtKB:Q70Z53",
  "gene_symbol": "FRA10AC1",
  "term_label": "phosphatase activity",
  "gene_name": "Protein FRA10AC1"
}